{
  "gene_name": "General transcription factor IIH subunit 4",
  "term_label": "transcription factor TFIIH core complex",
  "term_id": "GO:0000439",
  "gene_symbol": "GTF2H4",
  "gene": "UniProtKB:Q92759"
}